{
  "gene_symbol": "OXT",
  "gene": "UniProtKB:P01178",
  "term_label": "positive regulation of uterine smooth muscle contraction",
  "gene_name": "Oxytocin-neurophysin 1",
  "term_id": "GO:0070474"
}